regulation of oogonium development [GO:0075264] (biological process) Relationships: is a type of regulation of spore-bearing organ development [GO:0075260]; RO_0002211 GO:0075263 Subtypes: positive regulation of oogonium development [GO:0075265], negative regulation of oogonium development [GO:0075266] Sources: GOC:pamgo_curators Definition: Any process that modulates the frequency, rate or extent of oogonium development, a process that leads to the formation of a female gametangium of oomycetes, containing one or more gametes.